{
  "gene_symbol": "TNFSF13",
  "gene_name": "Tumor necrosis factor ligand superfamily member 13",
  "gene": "UniProtKB:O75888",
  "term_id": "GO:0048298",
  "term_label": "positive regulation of isotype switching to IgA isotypes"
}